{
  "term_id": "GO:0005737",
  "gene_symbol": "DCAF5",
  "gene": "UniProtKB:Q96JK2",
  "gene_name": "DDB1- and CUL4-associated factor 5",
  "term_label": "cytoplasm"
}